{
  "gene_name": "ADP-ribosylation factor-like protein 13A",
  "term_label": "non-motile cilium assembly",
  "gene": "UniProtKB:Q5H913",
  "term_id": "GO:1905515",
  "gene_symbol": "ARL13A"
}